{
  "term_label": "transcription corepressor activity",
  "term_id": "GO:0003714",
  "gene": "UniProtKB:Q9BQ87",
  "gene_name": "F-box-like_WD repeat-containing protein TBL1Y",
  "gene_symbol": "TBL1Y"
}